{
  "gene_symbol": "GPM6B",
  "gene": "UniProtKB:Q13491",
  "term_label": "axon development",
  "gene_name": "Neuronal membrane glycoprotein M6-b",
  "term_id": "GO:0061564"
}